{
  "gene_name": "Nuclear receptor subfamily 1 group D member 1",
  "gene_symbol": "NR1D1",
  "gene": "UniProtKB:P20393",
  "term_label": "cell differentiation",
  "term_id": "GO:0030154"
}